3,4-dihydroxyphthalate decarboxylase activity [GO:0047556] (molecular function) Relationships: is a type of carboxy-lyase activity [GO:0016831] Definition: Catalysis of the reaction: 3,4-dihydroxyphthalate + H+ = 3,4-dihydroxybenzoate + CO2. Sources: EC:4.1.1.69, RHEA:18601 Also known as: 3,4-dihydroxyphthalate 2-decarboxylase activity, 3,4-dihydroxyphthalate carboxy-lyase (3,4-dihydroxybenzoate-forming), 3,4-dihydroxyphthalate carboxy-lyase activity